negative regulation of vascular associated smooth muscle cell differentiation involved in phenotypic switching [GO:1905931] (biological process) Relationships: is a type of negative regulation of vascular associated smooth muscle cell differentiation [GO:1905064]; is a type of GO:1905916; is_a regulation of vascular associated smooth muscle cell differentiation involved in phenotypic switching [GO:1905930]; negatively regulates GO:1905420 Definition: Any process that stops, prevents or reduces the frequency, rate or extent of vascular smooth muscle cell differentiation involved in phenotypic switching. References: PMID:25089138 Sources: GOC:BHF, GOC:BHF_miRNA, GOC:TermGenie, GOC:rph, GO_REF:0000058 Also known as: down regulation of VSMC differentiation involved in phenotypic switching, down regulation of vascular associated smooth muscle cell differentiation involved in phenotypic switching, down regulation of vascular smooth muscle cell differentiation involved in phenotypic switching, down-regulation of VSMC differentiation involved in phenotypic switching, down-regulation of vascular associated smooth muscle cell differentiation involved in phenotypic switching, down-regulation of vascular smooth muscle cell differentiation involved in phenotypic switching, downregulation of VSMC differentiation involved in phenotypic switching, downregulation of vascular associated smooth muscle cell differentiation involved in phenotypic switching, downregulation of vascular smooth muscle cell differentiation involved in phenotypic switching, negative regulation of VSMC differentiation involved in phenotypic switching, negative regulation of vascular smooth muscle cell differentiation involved in phenotypic switching, inhibition of VSMC differentiation involved in phenotypic switching, inhibition of vascular associated smooth muscle cell differentiation involved in phenotypic switching, inhibition of vascular smooth muscle cell differentiation involved in phenotypic switching, down regulation of VSMC differentiation involved in phenotypic dimorphism, down regulation of vascular associated smooth muscle cell differentiation involved in phenotypic dimorphism, down regulation of vascular smooth muscle cell differentiation involved in phenotypic dimorphism, down-regulation of VSMC differentiation involved in phenotypic dimorphism, down-regulation of vascular associated smooth muscle cell differentiation involved in phenotypic dimorphism, down-regulation of vascular smooth muscle cell differentiation involved in phenotypic dimorphism, downregulation of VSMC differentiation involved in phenotypic dimorphism, downregulation of vascular associated smooth muscle cell differentiation involved in phenotypic dimorphism, downregulation of vascular smooth muscle cell differentiation involved in phenotypic dimorphism, inhibition of VSMC differentiation involved in phenotypic dimorphism, inhibition of vascular associated smooth muscle cell differentiation involved in phenotypic dimorphism, inhibition of vascular smooth muscle cell differentiation involved in phenotypic dimorphism, negative regulation of VSMC differentiation involved in phenotypic dimorphism, negative regulation of vascular associated smooth muscle cell differentiation involved in phenotypic dimorphism, negative regulation of vascular smooth muscle cell differentiation involved in phenotypic dimorphism